{
  "gene_symbol": "PSCA",
  "term_label": "acetylcholine receptor regulator activity",
  "term_id": "GO:0030548",
  "gene_name": "Prostate stem cell antigen",
  "gene": "UniProtKB:O43653"
}